nephric duct formation [GO:0072179] (biological process) Definition: The developmental process pertaining to the initial formation of a nephric duct. A nephric duct is a tube that drains a primitive kidney. Sources: GOC:mtg_kidney_jan10 Relationships: is a type of GO:0072175; is part of nephric duct morphogenesis [GO:0072178] Subtypes: mesonephric duct formation [GO:0072181]